CCR9 chemokine receptor binding [GO:0031734] (molecular function) Also known as: CCR9 chemokine receptor ligand Relationships: is a type of CCR chemokine receptor binding [GO:0048020] Sources: GOC:mah, GOC:nln Definition: Binding to a CCR9 chemokine receptor.